pyridoxine transmembrane transporter activity [GO:0031928] (molecular function) Sources: GOC:mah Also known as: pyridoxine transporter activity Definition: Enables the transfer of pyridoxine from one side of a membrane to the other. Pyridoxine, 2-methyl-3-hydroxy-4,5-bis(hydroxymethyl)pyridine, is one of the vitamin B6 compounds. Pyridoxal, pyridoxamine and pyridoxine are collectively known as vitamin B6, and are efficiently converted to the biologically active form of vitamin B6, pyridoxal phosphate. Relationships: is a type of transmembrane transporter activity [GO:0022857]; is part of pyridoxine transmembrane transport [GO:1903092]